{
  "gene_symbol": "PROSER1",
  "gene_name": "Proline and serine-rich protein 1",
  "gene": "UniProtKB:Q86XN7",
  "term_id": "UNKNOWN:0001",
  "term_label": "Unknown molecular function"
}